{
  "gene_symbol": "ATG16L2",
  "gene_name": "Protein Atg16l2",
  "term_label": "Unknown cellular component",
  "gene": "UniProtKB:Q8NAA4",
  "term_id": "UNKNOWN:0003"
}